{
  "gene_name": "Serine_threonine-protein kinase ULK1",
  "gene_symbol": "ULK1",
  "gene": "UniProtKB:O75385",
  "term_id": "GO:0034045",
  "term_label": "phagophore assembly site membrane"
}